{
  "term_id": "GO:0005509",
  "term_label": "calcium ion binding",
  "gene_name": "Group 10 secretory phospholipase A2",
  "gene_symbol": "PLA2G10",
  "gene": "UniProtKB:O15496"
}